{
  "gene": "UniProtKB:P60985",
  "term_id": "UNKNOWN:0001",
  "term_label": "Unknown molecular function",
  "gene_name": "Keratinocyte differentiation-associated protein",
  "gene_symbol": "KRTDAP"
}